{
  "term_id": "GO:0031490",
  "gene_symbol": "SBNO2",
  "term_label": "chromatin DNA binding",
  "gene_name": "Protein strawberry notch homolog 2",
  "gene": "UniProtKB:Q9Y2G9"
}